{
  "gene_symbol": "OMP",
  "gene": "UniProtKB:P47874",
  "term_label": "cytosol",
  "term_id": "GO:0005829",
  "gene_name": "Olfactory marker protein"
}